{
  "term_label": "ubiquitin protein ligase activity",
  "term_id": "GO:0061630",
  "gene": "UniProtKB:Q8TEJ3",
  "gene_symbol": "SH3RF3",
  "gene_name": "E3 ubiquitin-protein ligase SH3RF3"
}